{
  "gene": "UniProtKB:Q5TGU0",
  "gene_name": "Translocator protein 2",
  "term_id": "UNKNOWN:0001",
  "gene_symbol": "TSPO2",
  "term_label": "Unknown molecular function"
}